{
  "term_label": "membrane",
  "gene_name": "Protein lifeguard 3",
  "term_id": "GO:0016020",
  "gene": "UniProtKB:Q969X1",
  "gene_symbol": "TMBIM1"
}